{
  "gene_symbol": "FADS1",
  "gene_name": "Acyl-CoA (8-3)-desaturase",
  "gene": "UniProtKB:O60427",
  "term_label": "lipid metabolic process",
  "term_id": "GO:0006629"
}